antibiotic catabolic process [GO:0017001] (BP) Definition: The chemical reactions and pathways resulting in the breakdown of antibiotic, a substance produced by or derived from certain fungi, bacteria, and other organisms, that can destroy or inhibit the growth of other microorganisms. Sources: GOC:go_curators Also known as: antibiotic breakdown, antibiotic catabolism, antibiotic degradation Relationships: is a type of catabolic process [GO:0009056]; is a type of antibiotic metabolic process [GO:0016999] Subtypes: aminoglycoside antibiotic catabolic process [GO:0030649], peptide antibiotic catabolic process [GO:0030652], beta-lactam antibiotic catabolic process [GO:0030655], exogenous antibiotic catabolic process [GO:0042740], endogenous antibiotic catabolic process [GO:0042741]